{
  "gene_name": "Circadian locomoter output cycles protein kaput",
  "term_label": "DNA-binding transcription factor activity, RNA polymerase II-specific",
  "term_id": "GO:0000981",
  "gene": "UniProtKB:O15516",
  "gene_symbol": "CLOCK"
}